{
  "gene": "UniProtKB:P61769",
  "term_label": "MHC class II protein complex",
  "gene_name": "Beta-2-microglobulin",
  "gene_symbol": "B2M",
  "term_id": "GO:0042613"
}